{
  "gene_name": "RAS guanyl-releasing protein 1",
  "gene_symbol": "RASGRP1",
  "term_label": "positive regulation of natural killer cell mediated cytotoxicity",
  "gene": "UniProtKB:O95267",
  "term_id": "GO:0045954"
}